modulation of microtubule cytoskeleton involved in cerebral cortex radial glia guided migration [GO:0021815] (biological process) Definition: Rearrangements of the microtubule cytoskeleton that contribute to the movement of cells along radial glial cells as a component of the process of cerebral cortex glial-mediated radial migration. Subtypes: extension of a leading process involved in cell motility in cerebral cortex radial glia guided migration [GO:0021816] Also known as: modulation of microtubule cytoskeleton involved in cerebral cortex glial-mediated radial migration References: PMID:12626695 Sources: GOC:cls, GOC:dgh, GOC:dph, GOC:jid, GO_REF:0000021 Relationships: is a type of GO:0000226; is part of GO:0021814